L-DOPA receptor activity [GO:0035643] (molecular function) Relationships: is a type of neuropeptide receptor activity [GO:0008188]; has part L-DOPA binding [GO:0072544] References: PMID:18828673 Sources: Wikipedia:L-DOPA Definition: Combining with L-DOPA to initiate a change in cell activity. L-DOPA is the modified amino acid (2S)-2-amino-3-(3,4-dihydroxyphenyl) propanoic acid, and is the precursor to dopamine, norepinephrine (noradrenaline) and epinephrine. Also known as: L-beta-(3,4-Dihydroxyphenyl)alanine receptor activity